{
  "gene_name": "Actin-related protein 2_3 complex subunit 5-like protein",
  "gene": "UniProtKB:Q9BPX5",
  "term_label": "protein-macromolecule adaptor activity",
  "gene_symbol": "ARPC5L",
  "term_id": "GO:0030674"
}